{
  "gene_name": "Kelch-like protein 36",
  "gene_symbol": "KLHL36",
  "term_label": "Cul3-RING ubiquitin ligase complex",
  "gene": "UniProtKB:Q8N4N3",
  "term_id": "GO:0031463"
}